{
  "term_label": "3',5'-cyclic-AMP phosphodiesterase activity",
  "gene_symbol": "PDE4D",
  "term_id": "GO:0004115",
  "gene": "UniProtKB:Q08499",
  "gene_name": "cAMP-specific 3',5'-cyclic phosphodiesterase 4D"
}